positive regulation of autophagy in response to ER overload [GO:0034263] (BP) Relationships: is a type of GO:0006983; is a type of positive regulation of autophagy [GO:0010508] Also known as: autophagy in response to ER stress, autophagy in response to endoplasmic reticulum overload Definition: The process in which the accumulation of misfolded proteins in the endoplasmic reticulum triggers a response that positively regulates autophagy. Sources: GOC:mah